{
  "gene_symbol": "COPA",
  "term_id": "GO:0030126",
  "term_label": "COPI vesicle coat",
  "gene_name": "Coatomer subunit alpha",
  "gene": "UniProtKB:P53621"
}